{
  "term_id": "GO:0032435",
  "gene_symbol": "UBXN1",
  "gene": "UniProtKB:Q04323",
  "term_label": "negative regulation of proteasomal ubiquitin-dependent protein catabolic process",
  "gene_name": "UBX domain-containing protein 1"
}